mitogen-activated protein kinase p38 binding [GO:0048273] (molecular function) References: PMID:17827184 Sources: GOC:curators Also known as: MAPK p38 binding Definition: Binding to mitogen-activated protein kinase p38, an enzyme that catalyzes the transfer of phosphate from ATP to hydroxyl side chains on proteins in response to mitogen activation. Relationships: is_a mitogen-activated protein kinase binding [GO:0051019]